ecdysis, collagen and cuticulin-based cuticle [GO:0042395] (biological process) Definition: The shedding of the old collagen and cuticulin-based cuticle fragments during the molting cycle. Examples of this process are found in invertebrates. Relationships: is a type of molting cycle process [GO:0022404]; is part of GO:0018996 Sources: GOC:jl, GOC:mtg_sensu